{
  "term_id": "GO:0005737",
  "gene": "UniProtKB:Q86XT4",
  "gene_name": "E3 ubiquitin-protein ligase TRIM50",
  "term_label": "cytoplasm",
  "gene_symbol": "TRIM50"
}